antimicrobial humoral response [GO:0019730] (biological process) Definition: An immune response against microbes mediated through a body fluid. Examples of this process are seen in the antimicrobial humoral response of Drosophila melanogaster and Mus musculus. Subtypes: GO:0019731, antifungal humoral response [GO:0019732], antimicrobial humoral immune response mediated by antimicrobial peptide [GO:0061844] Relationships: is a type of humoral immune response [GO:0006959]; is a type of defense response to symbiont [GO:0140546] Sources: GOC:go_curators, GOC:mtg_sensu Regulation: regulated by regulation of antimicrobial humoral response [GO:0002759]; positively regulated by positive regulation of antimicrobial humoral response [GO:0002760]; RO_0002212 by negative regulation of antimicrobial humoral response [GO:0008348]